Golgi cisterna membrane [GO:0032580] (cellular component) Also known as: Golgi apparatus cisterna membrane, Golgi stack membrane Subtypes: GO:1990674, Golgi medial cisterna membrane [GO:1990675], GO:1990676 Relationships: is a type of organelle membrane [GO:0031090]; is part of Golgi cisterna [GO:0031985] Sources: GOC:ecd, GOC:mah Definition: The lipid bilayer surrounding any of the thin, flattened compartments that form the central portion of the Golgi complex.